{
  "gene": "UniProtKB:Q9Y6R1",
  "term_id": "GO:0051453",
  "gene_symbol": "SLC4A4",
  "gene_name": "Electrogenic sodium bicarbonate cotransporter 1",
  "term_label": "regulation of intracellular pH"
}